{
  "term_id": "GO:0005634",
  "gene": "UniProtKB:O94983",
  "gene_name": "Calmodulin-binding transcription activator 2",
  "term_label": "nucleus",
  "gene_symbol": "CAMTA2"
}